{
  "gene_symbol": "CASP10",
  "term_id": "GO:0004197",
  "gene": "UniProtKB:Q92851",
  "gene_name": "Caspase-10",
  "term_label": "cysteine-type endopeptidase activity"
}